{
  "gene": "UniProtKB:Q6ZNC4",
  "term_id": "GO:0006357",
  "term_label": "regulation of transcription by RNA polymerase II",
  "gene_symbol": "ZNF704",
  "gene_name": "Zinc finger protein 704"
}